{
  "term_id": "GO:0030154",
  "gene_symbol": "NR2E1",
  "gene_name": "Nuclear receptor subfamily 2 group E member 1",
  "term_label": "cell differentiation",
  "gene": "UniProtKB:Q9Y466"
}